{
  "gene_symbol": "ENTR1",
  "gene": "UniProtKB:Q96C92",
  "gene_name": "Endosome-associated-trafficking regulator 1",
  "term_label": "regulation of cytokinesis",
  "term_id": "GO:0032465"
}